{
  "gene": "UniProtKB:Q9H4H8",
  "term_id": "GO:0007165",
  "gene_name": "Protein FAM83D",
  "term_label": "signal transduction",
  "gene_symbol": "FAM83D"
}